{
  "term_label": "negative regulation of apoptotic process",
  "gene": "UniProtKB:P04792",
  "gene_name": "Heat shock protein beta-1",
  "term_id": "GO:0043066",
  "gene_symbol": "HSPB1"
}